{
  "gene_name": "T cell receptor alpha joining 59 (non-functional) (Fragment)",
  "gene": "UniProtKB:A0A075B6V9",
  "term_id": "UNKNOWN:0001",
  "term_label": "Unknown molecular function",
  "gene_symbol": "TRAJ59"
}